{
  "term_label": "vascular endothelial growth factor receptor activity",
  "term_id": "GO:0005021",
  "gene_symbol": "FLT4",
  "gene_name": "Vascular endothelial growth factor receptor 3",
  "gene": "UniProtKB:P35916"
}